AMP transport [GO:0080121] (biological process) Relationships: is_a organic cation transport [GO:0015695]; is_a GO:0015711; is a type of purine ribonucleotide transport [GO:0015868]; is a type of adenine nucleotide transport [GO:0051503] Definition: The directed movement of AMP, adenosine monophosphate, into, out of or within a cell, or between cells, by means of some agent such as a transporter or pore. Also known as: adenosine monophosphate transport References: PMID:18923018